interleukin-22 production [GO:0032626] (biological process) Definition: The appearance of interleukin-22 due to biosynthesis or secretion following a cellular stimulus, resulting in an increase in its intracellular or extracellular levels. Sources: GOC:mah Also known as: IL-22 production, IL22 production, ILTIF production, ZCYTO18 production, interleukin-22 biosynthetic process, interleukin-22 secretion Regulation: RO_0002211 by GO:0032666; negatively regulated by GO:0032706; positively regulated by positive regulation of interleukin-22 production [GO:0032746] Relationships: is_a cytokine production [GO:0001816]